{
  "term_label": "plasma membrane",
  "gene_name": "Sphingosine 1-phosphate receptor 1",
  "gene_symbol": "S1PR1",
  "term_id": "GO:0005886",
  "gene": "UniProtKB:P21453"
}